{
  "gene_symbol": "PNPLA1",
  "term_label": "lipid droplet",
  "term_id": "GO:0005811",
  "gene_name": "Omega-hydroxyceramide transacylase",
  "gene": "UniProtKB:Q8N8W4"
}